{
  "gene_symbol": "TRAF5",
  "term_label": "regulation of canonical NF-kappaB signal transduction",
  "term_id": "GO:0043122",
  "gene": "UniProtKB:O00463",
  "gene_name": "TNF receptor-associated factor 5"
}